{
  "gene": "UniProtKB:Q9H267",
  "gene_symbol": "VPS33B",
  "term_id": "GO:0005764",
  "term_label": "lysosome",
  "gene_name": "Vacuolar protein sorting-associated protein 33B"
}